{
  "term_label": "transcription regulator complex",
  "term_id": "GO:0005667",
  "gene": "UniProtKB:Q9Y2N7",
  "gene_name": "Hypoxia-inducible factor 3-alpha",
  "gene_symbol": "HIF3A"
}